{
  "gene_symbol": "KASH5",
  "term_label": "lateral element",
  "gene": "UniProtKB:Q8N6L0",
  "term_id": "GO:0000800",
  "gene_name": "Protein KASH5"
}